{
  "term_id": "GO:0005509",
  "term_label": "calcium ion binding",
  "gene_name": "Calmodulin-2",
  "gene_symbol": "CALM2",
  "gene": "UniProtKB:P0DP24"
}